{
  "gene": "UniProtKB:P52306",
  "term_id": "UNKNOWN:0002",
  "gene_symbol": "RAP1GDS1",
  "term_label": "Unknown biological process",
  "gene_name": "Rap1 GTPase-GDP dissociation stimulator 1"
}